{
  "gene_symbol": "ZNF236",
  "term_label": "regulation of transcription by RNA polymerase II",
  "gene_name": "Zinc finger protein 236",
  "term_id": "GO:0006357",
  "gene": "UniProtKB:Q9UL36"
}